{
  "gene_symbol": "SYT13",
  "gene": "UniProtKB:Q7L8C5",
  "term_id": "GO:2000300",
  "gene_name": "Synaptotagmin-13",
  "term_label": "regulation of synaptic vesicle exocytosis"
}